{
  "gene": "UniProtKB:P19532",
  "gene_name": "Transcription factor E3",
  "gene_symbol": "TFE3",
  "term_label": "DNA-binding transcription factor activity, RNA polymerase II-specific",
  "term_id": "GO:0000981"
}